{
  "gene_name": "Alpha-actinin-2",
  "term_id": "GO:0055001",
  "gene_symbol": "ACTN2",
  "gene": "UniProtKB:P35609",
  "term_label": "muscle cell development"
}